response to hesperadin [GO:1901595] (BP) Sources: GOC:TermGenie Subtypes: cellular response to hesperadin [GO:0072763] Definition: Any process that results in a change in state or activity of a cell or an organism (in terms of movement, secretion, enzyme production, gene expression, etc.) as a result of a hesperadin stimulus. Relationships: is a type of response to amine [GO:0014075]; is a type of response to oxygen-containing compound [GO:1901700]